{
  "gene": "UniProtKB:O95760",
  "gene_name": "Interleukin-33",
  "term_label": "positive regulation of cytokine production",
  "term_id": "GO:0001819",
  "gene_symbol": "IL33"
}